viral exocytosis [GO:0046754] (BP) Relationships: is a type of non-lytic viral release [GO:0046753] Definition: The exit of a fully formed virion particles from the host cell by exocytosis via a host vesicle. Also known as: viral egress by exocytosis References: PMID:33157038 Sources: ISBN:0072370319